{
  "gene": "UniProtKB:Q16558",
  "term_id": "GO:0015459",
  "gene_name": "Calcium-activated potassium channel subunit beta-1",
  "gene_symbol": "KCNMB1",
  "term_label": "potassium channel regulator activity"
}